{
  "gene_symbol": "RASA4",
  "gene_name": "Ras GTPase-activating protein 4",
  "term_id": "GO:0005096",
  "gene": "UniProtKB:O43374",
  "term_label": "GTPase activator activity"
}